double-strand break repair via single-strand annealing, removal of nonhomologous ends [GO:0000736] (biological process) References: PMID:10357855 Regulation: regulated by regulation of double-strand break repair via single-strand annealing, removal of nonhomologous ends [GO:1903776] Relationships: is a type of removal of nonhomologous ends [GO:0000735]; is part of GO:0045002 Definition: During DSBR via single-strand annealing, the removal of nonhomologous sequences at the broken 3' single-strand DNA end before DNA repair synthesis can occur.